{
  "gene": "UniProtKB:Q6ZUS5",
  "gene_name": "Coiled-coil domain-containing protein 121",
  "gene_symbol": "CCDC121",
  "term_id": "UNKNOWN:0002",
  "term_label": "Unknown biological process"
}